{
  "term_id": "GO:0045910",
  "term_label": "negative regulation of DNA recombination",
  "gene_name": "Putative spermatid-specific linker histone H1-like protein",
  "gene_symbol": "H1-9P",
  "gene": "UniProtKB:P60008"
}